{
  "gene": "UniProtKB:Q9NYG2",
  "gene_name": "Palmitoyltransferase ZDHHC3",
  "term_label": "regulation of G protein-coupled receptor signaling pathway",
  "term_id": "GO:0008277",
  "gene_symbol": "ZDHHC3"
}